{
  "term_label": "keratin filament",
  "gene": "UniProtKB:Q14533",
  "gene_name": "Keratin, type II cuticular Hb1",
  "gene_symbol": "KRT81",
  "term_id": "GO:0045095"
}